tyrocidine biosynthetic process [GO:1901904] (biological process) Definition: The chemical reactions and pathways resulting in the formation of tyrocidine. References: PMID:9352938 Sources: GOC:TermGenie, GOC:yaf, UniPathway:UPA00180 Also known as: tyrocidine anabolism, tyrocidine biosynthesis, tyrocidine formation, tyrocidine synthesis Relationships: is a type of biosynthetic process [GO:0009058]